positive regulation of G2/M transition of mitotic cell cycle [GO:0010971] (BP) Definition: Any signaling pathway that activates or increases the activity of a cell cycle cyclin-dependent protein kinase to modulate the switch from G2 phase to M phase of the mitotic cell cycle. Also known as: positive regulation of mitotic entry, positive regulation of cyclin-dependent protein serine/threonine kinase activity involved in G2/M transition of mitotic cell cycle Relationships: is_a regulation of G2/M transition of mitotic cell cycle [GO:0010389]; is a type of positive regulation of mitotic cell cycle phase transition [GO:1901992]; is a type of positive regulation of cell cycle G2/M phase transition [GO:1902751]; positively regulates G2/M transition of mitotic cell cycle [GO:0000086] Subtypes: positive regulation of G2/M transition of mitotic cell cycle involved in cellular response to nitrogen starvation [GO:1905287] Sources: GOC:dph, GOC:mtg_cell_cycle, GOC:tb